erythro-3-hydroxyaspartate ammonia-lyase activity [GO:0047447] (molecular function) Relationships: is a type of ammonia-lyase activity [GO:0016841] Definition: Catalysis of the reaction: erythro-3-hydroxy-L-aspartate = NH3 + oxaloacetic acid. Sources: EC:4.3.1.20, MetaCyc:4.3.1.20-RXN Also known as: 3-hydroxyaspartate dehydratase activity, erythro-3-hydroxyaspartate dehydratase activity, erythro-3-hydroxy-L(s)-aspartate hydro-lyase (deaminating) activity, erythro-3-hydroxy-Ls-aspartate ammonia-lyase (oxaloacetate-forming), erythro-3-hydroxy-Ls-aspartate ammonia-lyase activity, erythro-3-hydroxy-Ls-aspartate hydro-lyase (deaminating), erythro-beta-hydroxyaspartate dehydratase activity